{
  "term_label": "dense core granule",
  "gene": "UniProtKB:P21579",
  "gene_symbol": "SYT1",
  "term_id": "GO:0031045",
  "gene_name": "Synaptotagmin-1"
}